16-alpha-hydroxygypsogenate-UDP-glucosyltransferase activity [GO:0102937] (molecular function) Relationships: is a type of hexosyltransferase activity [GO:0016758] Sources: GOC:pz Definition: Catalysis of the reaction: UDP-alpha-D-glucose + 16-alpha-hydroxygypsogenate = 16-alpha-hydroxygypsogenate-28-beta-D-glucoside + UDP.